{
  "gene_symbol": "SCIN",
  "gene": "UniProtKB:Q9Y6U3",
  "term_label": "actin filament severing",
  "gene_name": "Scinderin",
  "term_id": "GO:0051014"
}